{
  "term_label": "Unknown molecular function",
  "gene": "UniProtKB:A6NES4",
  "gene_symbol": "MROH2A",
  "gene_name": "Maestro heat-like repeat-containing protein family member 2A",
  "term_id": "UNKNOWN:0001"
}